{
  "gene_name": "Claudin-5",
  "term_id": "GO:0005886",
  "gene": "UniProtKB:O00501",
  "gene_symbol": "CLDN5",
  "term_label": "plasma membrane"
}